RNA polymerase II CTD heptapeptide repeat S2 phosphatase activity [GO:0180006] (molecular function) Definition: Catalysis of the reaction: RNA polymerase II large subunit CTD heptapeptide repeat--phospho-L-serine (consensus YSPTSPS)(position 2) + H2O = RNA polymerase II large subunit + phosphate. Relationships: is a type of RNA polymerase II CTD heptapeptide repeat phosphatase activity [GO:0008420] Also known as: RNA polymerase II C-terminal domain S2 phosphatase activity References: PMID:22622228